{
  "gene_name": "TGF-beta receptor type-1",
  "term_id": "GO:0046332",
  "gene": "UniProtKB:P36897",
  "term_label": "SMAD binding",
  "gene_symbol": "TGFBR1"
}